norepinephrine metabolic process [GO:0042415] (biological process) Relationships: is a type of GO:0006584 Also known as: levarterenol metabolic process, levarterenol metabolism, noradrenaline metabolic process, noradrenaline metabolism, norepinephrine metabolism Sources: GOC:jl, ISBN:0198506732 Subtypes: norepinephrine biosynthetic process [GO:0042421], norepinephrine catabolic process [GO:0042422] Definition: The chemical reactions and pathways involving norepinephrine, a hormone secreted by the adrenal medulla, and a neurotransmitter in the sympathetic peripheral nervous system and in some tracts in the central nervous system. It is also the demethylated biosynthetic precursor of epinephrine.